beta-alanine metabolic process [GO:0019482] (biological process) Sources: GOC:jl, ISBN:0198506732 Subtypes: beta-alanine biosynthetic process [GO:0019483], beta-alanine catabolic process [GO:0019484] Definition: The chemical reactions and pathways involving beta-alanine (3-aminopropanoic acid), an achiral amino acid and an isomer of alanine. It occurs free (e.g. in brain) and in combination (e.g. in pantothenate) but it is not a constituent of proteins. Also known as: beta-alanine metabolism Relationships: is a type of non-proteinogenic amino acid metabolic process [GO:0170041]